{
  "gene_symbol": "TMEM98",
  "term_id": "UNKNOWN:0002",
  "term_label": "Unknown biological process",
  "gene_name": "Transmembrane protein 98",
  "gene": "UniProtKB:Q9Y2Y6"
}